{
  "term_label": "Unknown molecular function",
  "gene_name": "Immunoglobulin lambda variable 3-1",
  "gene_symbol": "IGLV3-1",
  "term_id": "UNKNOWN:0001",
  "gene": "UniProtKB:P01715"
}